{
  "gene_symbol": "EDC4",
  "term_id": "GO:0000932",
  "gene_name": "Enhancer of mRNA-decapping protein 4",
  "gene": "UniProtKB:Q6P2E9",
  "term_label": "P-body"
}